stress fiber assembly [GO:0043149] (biological process) Definition: The aggregation, arrangement and bonding together of a set of components to form a stress fiber. A stress fiber is a contractile actin filament bundle that consists of short actin filaments with alternating polarity. References: PMID:16651381 Sources: GOC:go_curators, GOC:mah Also known as: actin cable assembly, actin cable formation, stress fibre biosynthesis, stress fibre formation Relationships: is a type of contractile actin filament bundle assembly [GO:0030038]; is a type of actomyosin structure organization [GO:0031032] Regulation: regulated by regulation of stress fiber assembly [GO:0051492]; RO_0002213 by positive regulation of stress fiber assembly [GO:0051496]; RO_0002212 by GO:0051497